{
  "term_id": "GO:0005634",
  "gene": "UniProtKB:P51955",
  "gene_name": "Serine_threonine-protein kinase Nek2",
  "term_label": "nucleus",
  "gene_symbol": "NEK2"
}